regulation of fever generation by prostaglandin biosynthetic process [GO:0100008] (biological process) Regulation: regulated by GO:0071809 Relationships: is_a prostaglandin biosynthetic process [GO:0001516]; regulates GO:0001660 Sources: GOC:cjm, GOC:obol Subtypes: positive regulation of fever generation by prostaglandin biosynthetic process [GO:0100010] Definition: Any prostaglandin biosynthetic process process that regulates fever generation.